{
  "gene_symbol": "STX10",
  "term_label": "intracellular protein transport",
  "gene_name": "Syntaxin-10",
  "term_id": "GO:0006886",
  "gene": "UniProtKB:O60499"
}